{
  "term_id": "GO:0005262",
  "gene": "UniProtKB:Q9NQA5",
  "term_label": "calcium channel activity",
  "gene_name": "Transient receptor potential cation channel subfamily V member 5",
  "gene_symbol": "TRPV5"
}